{
  "gene_name": "F-box_WD repeat-containing protein 12",
  "term_id": "UNKNOWN:0003",
  "term_label": "Unknown cellular component",
  "gene": "UniProtKB:Q6X9E4",
  "gene_symbol": "FBXW12"
}